{
  "gene": "UniProtKB:Q99523",
  "gene_symbol": "SORT1",
  "gene_name": "Sortilin",
  "term_id": "GO:0016050",
  "term_label": "vesicle organization"
}